lytic vacuole within protein storage vacuole [GO:0000327] (cellular component) References: PMID:11739490 Definition: A membrane-bounded compartment containing crystals of phytic acid and proteins characteristic of a lytic vacuole, found within a storage vacuole. Relationships: is a type of GO:0000323; is part of protein storage vacuole [GO:0000326]